{
  "gene_symbol": "NAP1L3",
  "term_label": "nucleus",
  "gene": "UniProtKB:Q99457",
  "gene_name": "Nucleosome assembly protein 1-like 3",
  "term_id": "GO:0005634"
}